gamma-delta T cell proliferation [GO:0046630] (BP) Sources: GOC:ai Subtypes: gamma-delta T cell proliferation involved in immune response [GO:0002311] Relationships: is_a T cell proliferation [GO:0042098]; is a type of gamma-delta T cell activation [GO:0046629] Regulation: regulated by regulation of gamma-delta T cell proliferation [GO:0046646]; negatively regulated by negative regulation of gamma-delta T cell proliferation [GO:0046647]; positively regulated by positive regulation of gamma-delta T cell proliferation [GO:0046648] Definition: The expansion of a gamma-delta T cell population by cell division. Also known as: gamma-delta T lymphocyte proliferation, gamma-delta T-cell proliferation, gamma-delta T-lymphocyte proliferation